{
  "gene": "UniProtKB:Q9NQL9",
  "gene_symbol": "DMRT3",
  "term_label": "DNA-binding transcription factor activity, RNA polymerase II-specific",
  "term_id": "GO:0000981",
  "gene_name": "Doublesex- and mab-3-related transcription factor 3"
}